regulation of compound eye pigmentation [GO:0048076] (biological process) Definition: Any process that modulates the frequency, rate or extent of establishment of a pattern of pigment in the compound eye. Subtypes: negative regulation of compound eye pigmentation [GO:0048077], positive regulation of compound eye pigmentation [GO:0048078] Sources: GOC:jid Relationships: is a type of GO:0048073; regulates compound eye pigmentation [GO:0048072]